detection of glucose [GO:0051594] (biological process) Sources: GOC:ai Definition: The series of events in which a glucose stimulus is received by a cell and converted into a molecular signal. Regulation: regulated by GO:2000970; negatively regulated by negative regulation of detection of glucose [GO:2000971]; positively regulated by positive regulation of detection of glucose [GO:2000972] Also known as: glucose detection, glucose perception, glucose sensing Relationships: is a type of detection of hexose stimulus [GO:0009732]; is a type of GO:0009749